negative regulation of brassinosteroid biosynthetic process [GO:0010423] (biological process) Definition: Any process that stops, prevents, or reduces the frequency, rate or extent of the chemical reactions and pathways resulting in the formation of brassinosteroids. References: PMID:16857903 Relationships: is a type of regulation of brassinosteroid biosynthetic process [GO:0010422]; is a type of negative regulation of steroid hormone biosynthetic process [GO:0090032]; negatively regulates brassinosteroid biosynthetic process [GO:0016132]